{
  "term_label": "nucleus",
  "gene_symbol": "THRSP",
  "gene": "UniProtKB:Q92748",
  "gene_name": "Thyroid hormone-inducible hepatic protein",
  "term_id": "GO:0005634"
}